{
  "gene_symbol": "RBM4B",
  "gene_name": "RNA-binding protein 4B",
  "term_label": "regulation of alternative mRNA splicing, via spliceosome",
  "gene": "UniProtKB:Q9BQ04",
  "term_id": "GO:0000381"
}